{
  "term_id": "GO:0004984",
  "gene_symbol": "OR4C5",
  "gene_name": "Olfactory receptor 4C5",
  "gene": "UniProtKB:Q8NGB2",
  "term_label": "olfactory receptor activity"
}